negative regulation of nematode larval development [GO:0061064] (biological process) Sources: GOC:dph, GOC:kmv Subtypes: negative regulation of vulval development [GO:0040027], negative regulation of dauer larval development [GO:0061067], negative regulation of nematode larval development, heterochronic [GO:0090446] Relationships: is a type of negative regulation of post-embryonic development [GO:0048581]; is a type of GO:0061062; negatively regulates GO:0002119 Definition: Any process that decreases the rate, frequency, or extent of nematode larval development, the process whose specific outcome is the progression of the nematode larva over time, from its formation to the mature structure. Nematode larval development begins with the newly hatched first-stage larva (L1) and ends with the end of the last larval stage (for example the fourth larval stage (L4) in C. elegans). Each stage of nematode larval development is characterized by proliferation of specific cell lineages and an increase in body size without alteration of the basic body plan. Nematode larval stages are separated by molts in which each stage-specific exoskeleton, or cuticle, is shed and replaced anew.